{
  "term_label": "receptor signaling protein tyrosine kinase activator activity",
  "gene": "UniProtKB:Q6UXT8",
  "gene_symbol": "ALKAL1",
  "gene_name": "ALK and LTK ligand 1",
  "term_id": "GO:0030298"
}